{
  "gene_symbol": "CDHR3",
  "term_id": "GO:0016477",
  "gene_name": "Cadherin-related family member 3",
  "gene": "UniProtKB:Q6ZTQ4",
  "term_label": "cell migration"
}